programmed cell death in response to reactive oxygen species [GO:0097468] (biological process) Definition: Cell death resulting from activation of endogenous cellular processes and occurring as a result of a reactive oxygen species stimulus. Reactive oxygen species include singlet oxygen, superoxide, and oxygen free radicals. Relationships: is_a GO:0012501; is part of cellular response to reactive oxygen species [GO:0034614] Subtypes: GO:0010343, hydrogen peroxide-mediated programmed cell death [GO:0010421] Also known as: PCD in response to oxidative stress, programmed cell death in response to oxidative stress, PCD in response to reactive oxygen species, reactive oxygen species-mediated PCD, reactive oxygen species-mediated programmed cell death Sources: GOC:mtg_apoptosis